{
  "gene": "UniProtKB:O95249",
  "term_id": "GO:0048219",
  "term_label": "inter-Golgi cisterna vesicle-mediated transport",
  "gene_symbol": "GOSR1",
  "gene_name": "Golgi SNAP receptor complex member 1"
}